{
  "gene": "UniProtKB:O95965",
  "gene_name": "Integrin beta-like protein 1",
  "gene_symbol": "ITGBL1",
  "term_label": "integrin binding",
  "term_id": "GO:0005178"
}